{
  "gene": "UniProtKB:P07333",
  "term_label": "positive regulation of cell migration",
  "term_id": "GO:0030335",
  "gene_name": "Macrophage colony-stimulating factor 1 receptor",
  "gene_symbol": "CSF1R"
}